{
  "gene": "UniProtKB:Q9Y5Z9",
  "gene_symbol": "UBIAD1",
  "term_label": "prenyltransferase activity",
  "term_id": "GO:0004659",
  "gene_name": "UbiA prenyltransferase domain-containing protein 1"
}